negative regulation of high voltage-gated calcium channel activity [GO:1901842] (biological process) Also known as: down regulation of high voltage gated calcium channel activity, down regulation of high voltage-dependent calcium channel activity, down regulation of high voltage-gated calcium channel activity, down-regulation of high voltage gated calcium channel activity, down-regulation of high voltage-dependent calcium channel activity, down-regulation of high voltage-gated calcium channel activity, downregulation of high voltage gated calcium channel activity, downregulation of high voltage-dependent calcium channel activity, downregulation of high voltage-gated calcium channel activity, inhibition of high voltage gated calcium channel activity, inhibition of high voltage-dependent calcium channel activity, negative regulation of high voltage gated calcium channel activity, negative regulation of high voltage-dependent calcium channel activity, inhibition of high voltage-gated calcium channel activity References: PMID:12754254 Sources: GOC:BHF, GOC:TermGenie, GOC:rl Definition: Any process that stops, prevents or reduces the frequency, rate or extent of high voltage-gated calcium channel activity. Relationships: is a type of negative regulation of voltage-gated calcium channel activity [GO:1901386]; negatively regulates high voltage-gated calcium channel activity [GO:0008331]